{
  "gene_symbol": "CDH9",
  "gene": "UniProtKB:Q9ULB4",
  "term_label": "cell morphogenesis",
  "term_id": "GO:0000902",
  "gene_name": "Cadherin-9"
}